{
  "gene": "UniProtKB:P20062",
  "term_id": "GO:0005615",
  "gene_symbol": "TCN2",
  "term_label": "extracellular space",
  "gene_name": "Transcobalamin-2"
}